{
  "term_id": "GO:0005829",
  "gene": "UniProtKB:Q9Y484",
  "gene_name": "WD repeat domain phosphoinositide-interacting protein 4",
  "gene_symbol": "WDR45",
  "term_label": "cytosol"
}